ketogluconate biosynthetic process [GO:0046180] (biological process) Relationships: is_a aldonic acid biosynthetic process [GO:0046175] Subtypes: keto-D-gluconate biosynthetic process [GO:0046179] Also known as: ketogluconate anabolism, ketogluconate biosynthesis, ketogluconate formation, ketogluconate synthesis Sources: ISBN:0198506732 Definition: The chemical reactions and pathways resulting in the formation of ketogluconate, the anion of ketogluconic acid, an aldonic acid derived from glucose containing a ketonic carbonyl group.